{
  "term_id": "GO:0005886",
  "gene_symbol": "ARAP1",
  "gene_name": "Arf-GAP with Rho-GAP domain, ANK repeat and PH domain-containing protein 1",
  "gene": "UniProtKB:Q96P48",
  "term_label": "plasma membrane"
}